{
  "gene_symbol": "NUP54",
  "gene": "UniProtKB:Q7Z3B4",
  "gene_name": "Nucleoporin p54",
  "term_label": "NLS-bearing protein import into nucleus",
  "term_id": "GO:0006607"
}